{
  "term_label": "zinc ion binding",
  "term_id": "GO:0008270",
  "gene_name": "Integrin beta-1-binding protein 2",
  "gene": "UniProtKB:Q9UKP3",
  "gene_symbol": "ITGB1BP2"
}